{
  "gene": "UniProtKB:P08069",
  "gene_symbol": "IGF1R",
  "term_id": "GO:0005886",
  "term_label": "plasma membrane",
  "gene_name": "Insulin-like growth factor 1 receptor"
}